{
  "term_label": "signaling receptor binding",
  "term_id": "GO:0005102",
  "gene_name": "Protein cornichon homolog 2",
  "gene": "UniProtKB:Q6PI25",
  "gene_symbol": "CNIH2"
}